{
  "term_id": "GO:0034041",
  "gene_name": "ATP-binding cassette sub-family G member 4",
  "gene_symbol": "ABCG4",
  "gene": "UniProtKB:Q9H172",
  "term_label": "ABC-type sterol transporter activity"
}